{
  "gene_name": "Leiomodin-1",
  "term_label": "striated muscle thin filament",
  "term_id": "GO:0005865",
  "gene": "UniProtKB:P29536",
  "gene_symbol": "LMOD1"
}